{
  "gene": "UniProtKB:Q00587",
  "gene_symbol": "CDC42EP1",
  "term_label": "cytoplasm",
  "term_id": "GO:0005737",
  "gene_name": "Cdc42 effector protein 1"
}